{
  "gene": "UniProtKB:Q96EY1",
  "gene_symbol": "DNAJA3",
  "term_label": "protein kinase binding",
  "term_id": "GO:0019901",
  "gene_name": "DnaJ homolog subfamily A member 3, mitochondrial"
}